{
  "gene": "UniProtKB:Q15172",
  "term_label": "nucleus",
  "term_id": "GO:0005634",
  "gene_symbol": "PPP2R5A",
  "gene_name": "Serine_threonine-protein phosphatase 2A 56 kDa regulatory subunit alpha isoform"
}